{
  "term_label": "kinesin binding",
  "term_id": "GO:0019894",
  "gene_symbol": "AP1AR",
  "gene": "UniProtKB:Q63HQ0",
  "gene_name": "AP-1 complex-associated regulatory protein"
}